{
  "gene_name": "Keratin, type II cytoskeletal 6C",
  "term_label": "keratin filament",
  "term_id": "GO:0045095",
  "gene": "UniProtKB:P48668",
  "gene_symbol": "KRT6C"
}